primary cell septum biogenesis [GO:0031671] (biological process) Relationships: is a type of GO:0044085; is a type of mitotic cytokinetic process [GO:1902410]; is part of mitotic division septum assembly [GO:0140278] Regulation: regulated by regulation of primary cell septum biogenesis [GO:1905756]; negatively regulated by negative regulation of primary cell septum biogenesis [GO:1905757]; positively regulated by positive regulation of primary cell septum biogenesis [GO:1905758] Sources: GOC:jl Definition: A cellular process that results in the biosynthesis of constituent macromolecules, assembly, and arrangement of constituent parts of a primary cell septum following nuclear division.